{
  "term_label": "positive regulation of mitotic cell cycle",
  "term_id": "GO:0045931",
  "gene_name": "Coiled-coil domain-containing protein 57",
  "gene_symbol": "CCDC57",
  "gene": "UniProtKB:Q2TAC2"
}